{
  "gene": "UniProtKB:Q9UK97",
  "term_id": "GO:0031146",
  "term_label": "SCF-dependent proteasomal ubiquitin-dependent protein catabolic process",
  "gene_name": "F-box only protein 9",
  "gene_symbol": "FBXO9"
}